{
  "term_id": "UNKNOWN:0002",
  "term_label": "Unknown biological process",
  "gene": "UniProtKB:Q9NXR8",
  "gene_name": "Inhibitor of growth protein 3",
  "gene_symbol": "ING3"
}